response to interleukin-11 [GO:0071105] (biological process) Subtypes: GO:0071348 Also known as: response to IL-11 Relationships: is a type of response to cytokine [GO:0034097] Definition: Any process that results in a change in state or activity of a cell or an organism (in terms of movement, secretion, enzyme production, gene expression, etc.) as a result of an interleukin-11 stimulus. Sources: GOC:mah, GOC:yaf